{
  "gene_symbol": "TUBG1",
  "term_id": "GO:0005737",
  "term_label": "cytoplasm",
  "gene_name": "Tubulin gamma-1 chain",
  "gene": "UniProtKB:P23258"
}